{
  "gene_name": "Chordin-like protein 1",
  "term_label": "cell differentiation",
  "gene": "UniProtKB:Q9BU40",
  "gene_symbol": "CHRDL1",
  "term_id": "GO:0030154"
}